{
  "term_id": "GO:0008233",
  "gene_name": "Cilia- and flagella-associated protein 44",
  "gene": "UniProtKB:Q96MT7",
  "gene_symbol": "CFAP44",
  "term_label": "peptidase activity"
}